tRNA (5-methylaminomethyl-2-thiouridylate)(34)-methyltransferase activity [GO:0004808] (MF) Relationships: is a type of GO:0008757; is a type of GO:0016300 Also known as: tRNA (5-methylaminomethyl-2-thiouridylate)-methyltransferase activity, tRNA 5-methylaminomethyl-2-thiouridylate 5'-methyltransferase activity Sources: RHEA:19569 Definition: Catalysis of the reaction: 5-aminomethyl-2-thiouridine34 in tRNA + S-adenosyl-L-methionine = 5-methylaminomethyl-2-thiouridine34 in tRNA + H+ + S-adenosyl-L-homocysteine. This enzyme specifically adds the terminal methyl group of 5-[(methylamino)methyl]-2-thiouridylate.